{
  "term_id": "GO:0045087",
  "gene": "UniProtKB:Q96PH6",
  "term_label": "innate immune response",
  "gene_name": "Defensin beta 118",
  "gene_symbol": "DEFB118"
}